{
  "term_id": "GO:0033188",
  "term_label": "sphingomyelin synthase activity",
  "gene_symbol": "SGMS2",
  "gene": "UniProtKB:Q8NHU3",
  "gene_name": "Phosphatidylcholine:ceramide cholinephosphotransferase 2"
}